{
  "term_label": "determination of ventral identity",
  "gene_symbol": "AIDA",
  "gene": "UniProtKB:Q96BJ3",
  "term_id": "GO:0048264",
  "gene_name": "Axin interactor, dorsalization-associated protein"
}